endoplasmic reticulum quality control compartment [GO:0044322] (cellular component) References: PMID:11408579 Relationships: is a type of GO:0110165; is part of endoplasmic reticulum [GO:0005783] Also known as: ER quality control compartment, ERQC, ER-derived quality control compartment Definition: A subcompartment of the endoplasmic reticulum in which proteins with improper or incorrect folding accumulate. Enzymes in this compartment direct proteins with major folding problems to translocation to the cytosol and degradation, and proteins with minor folding problems to the ER, to interact with chaperon proteins.